{
  "gene_name": "Ras GTPase-activating-like protein IQGAP3",
  "gene": "UniProtKB:Q86VI3",
  "term_label": "mitotic actomyosin contractile ring assembly actin filament organization",
  "gene_symbol": "IQGAP3",
  "term_id": "GO:1903479"
}